{
  "term_id": "UNKNOWN:0002",
  "term_label": "Unknown biological process",
  "gene_symbol": "SPATA33",
  "gene_name": "Spermatogenesis-associated protein 33",
  "gene": "UniProtKB:Q96N06"
}